{
  "gene": "UniProtKB:P30953",
  "term_id": "GO:0007165",
  "term_label": "signal transduction",
  "gene_symbol": "OR1E1",
  "gene_name": "Olfactory receptor 1E1"
}